{
  "gene_name": "Ribonuclease pancreatic",
  "gene": "UniProtKB:P07998",
  "term_label": "defense response to Gram-positive bacterium",
  "gene_symbol": "RNASE1",
  "term_id": "GO:0050830"
}